{
  "gene": "UniProtKB:Q15005",
  "gene_symbol": "SPCS2",
  "term_id": "GO:0045047",
  "gene_name": "Signal peptidase complex subunit 2",
  "term_label": "protein targeting to ER"
}